regulation of cutin biosynthetic process [GO:1901957] (biological process) References: PMID:23243127 Sources: GOC:TermGenie, GOC:tb Subtypes: negative regulation of cutin biosynthetic process [GO:1901958], positive regulation of cutin biosynthetic process [GO:1901959] Also known as: regulation of cutin anabolism, regulation of cutin biosynthesis, regulation of cutin formation, regulation of cutin synthesis Definition: Any process that modulates the frequency, rate or extent of cutin biosynthetic process. Relationships: is a type of regulation of macromolecule biosynthetic process [GO:0010556]; regulates cutin biosynthetic process [GO:0010143]